all-trans-beta-apo-10'-carotenal cleavage oxygenase activity [GO:0102251] (molecular function) Relationships: is a type of oxidoreductase activity, acting on single donors with incorporation of molecular oxygen, incorporation of two atoms of oxygen [GO:0016702] Definition: Catalysis of the reaction: 10'-apo-beta-carotenal + O2 = 13-apo-beta-carotenone + 4-methylocta-2,4,6-trienedial. Sources: EC:1.13.11.70, GOC:pz